detection of peptidoglycan [GO:0032499] (biological process) Subtypes: GO:0032498 Sources: GOC:add, ISBN:0721601464 Relationships: is a type of detection of molecule of bacterial origin [GO:0032490]; is a type of response to peptidoglycan [GO:0032494] Definition: The series of events in which a peptidoglycan stimulus is received by a cell and converted into a molecular signal. Peptidoglycan is a bacterial cell wall macromolecule.